{
  "gene_symbol": "KIAA1210",
  "term_label": "Unknown molecular function",
  "gene_name": "Acrosomal protein KIAA1210",
  "gene": "UniProtKB:Q9ULL0",
  "term_id": "UNKNOWN:0001"
}